vacuolar proton-transporting V-type ATPase complex [GO:0016471] (CC) Subtypes: lysosomal proton-transporting V-type ATPase complex [GO:0046611] Relationships: is a type of proton-transporting V-type ATPase complex [GO:0033176]; is part of GO:0005774 Definition: A proton-transporting two-sector ATPase complex found in the vacuolar membrane, where it acts as a proton pump to mediate acidification of the vacuolar lumen. Also known as: vacuolar hydrogen-translocating V-type ATPase complex References: PMID:16449553 Sources: GOC:mah, ISBN:0716743663 Note: See also the cellular component terms 'vacuolar proton-transporting V-type ATPase, V1 domain ; GO:0000221' and 'vacuolar proton-transporting V-type ATPase, V0 domain ; GO:0000220' and the molecular function term 'hydrogen ion transporting ATPase activity, rotational mechanism ; GO:0046961'.